{
  "term_label": "Unknown biological process",
  "term_id": "UNKNOWN:0002",
  "gene_name": "Zinc finger protein 234",
  "gene_symbol": "ZNF234",
  "gene": "UniProtKB:Q14588"
}